{
  "gene": "UniProtKB:Q2TBC4",
  "term_label": "stress fiber",
  "gene_name": "Prickle-like protein 4",
  "gene_symbol": "PRICKLE4",
  "term_id": "GO:0001725"
}